{
  "gene_name": "Cytochrome P450 4F12",
  "term_label": "arachidonate metabolic process",
  "gene": "UniProtKB:Q9HCS2",
  "term_id": "GO:0019369",
  "gene_symbol": "CYP4F12"
}